{
  "gene_name": "Elongation factor G, mitochondrial",
  "term_id": "GO:0003924",
  "term_label": "GTPase activity",
  "gene": "UniProtKB:Q96RP9",
  "gene_symbol": "GFM1"
}